{
  "term_label": "Unknown molecular function",
  "gene": "UniProtKB:A0A6Q8PFQ6",
  "gene_symbol": "A0A6Q8PFQ6",
  "gene_name": "Uncharacterized protein",
  "term_id": "UNKNOWN:0001"
}